peptide receptor activity [GO:0001653] (molecular function) Also known as: endogenous peptide receptor activity, exogenous peptide receptor activity Subtypes: G protein-coupled peptide receptor activity [GO:0008528], natriuretic peptide receptor activity [GO:0016941], opioid growth factor receptor activity [GO:0140625] Definition: Combining with an extracellular or intracellular peptide to initiate a change in cell activity. Relationships: is a type of signaling receptor activity [GO:0038023]; has part peptide binding [GO:0042277] Sources: GOC:jl